{
  "gene": "UniProtKB:Q9NQX1",
  "gene_name": "PR domain zinc finger protein 5",
  "term_label": "negative regulation of DNA-templated transcription",
  "term_id": "GO:0045892",
  "gene_symbol": "PRDM5"
}